{
  "term_label": "titin binding",
  "gene_symbol": "TCAP",
  "gene": "UniProtKB:O15273",
  "gene_name": "Telethonin",
  "term_id": "GO:0031432"
}